{
  "term_label": "neuropeptide signaling pathway",
  "gene": "UniProtKB:P07492",
  "gene_symbol": "GRP",
  "term_id": "GO:0007218",
  "gene_name": "Gastrin-releasing peptide"
}